{
  "gene_symbol": "RAB3A",
  "gene_name": "Ras-related protein Rab-3A",
  "term_label": "acrosomal vesicle exocytosis",
  "gene": "UniProtKB:P20336",
  "term_id": "GO:0060478"
}